retina vasculature development in camera-type eye [GO:0061298] (biological process) Also known as: retinal vasculature development Definition: The process whose specific outcome is the progression of the vasculature of the retina over time, from its formation to the mature structure. Sources: GOC:BHF, GOC:dph Relationships: is a type of vasculature development [GO:0001944]; is part of retina development in camera-type eye [GO:0060041]